{
  "term_label": "vein smooth muscle contraction",
  "term_id": "GO:0014826",
  "gene_symbol": "EDN3",
  "gene": "UniProtKB:P14138",
  "gene_name": "Endothelin-3"
}